{
  "term_label": "epithelial cell differentiation",
  "term_id": "GO:0030855",
  "gene_name": "Keratin, type I cytoskeletal 27",
  "gene": "UniProtKB:Q7Z3Y8",
  "gene_symbol": "KRT27"
}